{
  "gene_name": "Heterogeneous nuclear ribonucleoprotein M",
  "term_label": "nucleus",
  "term_id": "GO:0005634",
  "gene_symbol": "HNRNPM",
  "gene": "UniProtKB:P52272"
}